cyclin-dependent protein serine/threonine kinase activator activity [GO:0061575] (molecular function) Relationships: is a type of GO:0016538; is a type of protein serine/threonine kinase activator activity [GO:0043539]; positively regulates GO:0004693 References: PMID:2569363, PMID:3322810 Sources: GOC:dph Also known as: cyclin-dependent protein kinase 5 activator activity Definition: Binds to and increases the activity of a cyclin-dependent protein serine/threonine kinase.